{
  "term_id": "GO:0045944",
  "term_label": "positive regulation of transcription by RNA polymerase II",
  "gene": "UniProtKB:P10243",
  "gene_name": "Myb-related protein A",
  "gene_symbol": "MYBL1"
}